{
  "gene_symbol": "RIDA",
  "term_id": "GO:0006402",
  "term_label": "mRNA catabolic process",
  "gene_name": "2-iminobutanoate_2-iminopropanoate deaminase",
  "gene": "UniProtKB:P52758"
}